vestibulospinal tract morphogenesis [GO:0021962] (biological process) Relationships: is a type of central nervous system projection neuron axonogenesis [GO:0021952] Definition: Generation of a long process of a CNS neuron, that carries efferent (outgoing) action potentials from the cell body in the vestibular nucleus of the pons towards target cells in the spinal cord. Sources: GOC:cls, GOC:dgh, GOC:dph, GOC:jid, GO_REF:0000021